{
  "gene_symbol": "B3GALT5",
  "term_id": "UNKNOWN:0002",
  "gene": "UniProtKB:Q9Y2C3",
  "term_label": "Unknown biological process",
  "gene_name": "Beta-1,3-galactosyltransferase 5"
}